{
  "term_label": "Unknown cellular component",
  "gene_symbol": "ZSCAN21",
  "gene_name": "Zinc finger and SCAN domain-containing protein 21",
  "gene": "UniProtKB:Q9Y5A6",
  "term_id": "UNKNOWN:0003"
}